amine catabolic process [GO:0009310] (BP) Relationships: is a type of GO:0009056; is a type of amine metabolic process [GO:0009308] Definition: The chemical reactions and pathways resulting in the breakdown of any organic compound that is weakly basic in character and contains an amino or a substituted amino group. Amines are called primary, secondary, or tertiary according to whether one, two, or three carbon atoms are attached to the nitrogen atom. Subtypes: biogenic amine catabolic process [GO:0042402], 2-aminobenzenesulfonate catabolic process [GO:0046230] Sources: GOC:jl, ISBN:0198506732 Also known as: amine breakdown, amine catabolism, amine degradation Regulation: RO_0002211 by regulation of amine catabolic process [GO:0033241]; negatively regulated by negative regulation of amine catabolic process [GO:0033242]; positively regulated by GO:0033243